{
  "gene": "UniProtKB:Q14397",
  "term_label": "intracellular glucose homeostasis",
  "gene_symbol": "GCKR",
  "term_id": "GO:0001678",
  "gene_name": "Glucokinase regulatory protein"
}